{
  "gene_name": "CDK5 regulatory subunit-associated protein 3",
  "term_id": "GO:0007346",
  "term_label": "regulation of mitotic cell cycle",
  "gene_symbol": "CDK5RAP3",
  "gene": "UniProtKB:Q96JB5"
}